{
  "gene_name": "2-oxoisovalerate dehydrogenase subunit alpha, mitochondrial",
  "term_id": "GO:0009083",
  "gene_symbol": "BCKDHA",
  "gene": "UniProtKB:P12694",
  "term_label": "branched-chain amino acid catabolic process"
}